coenzyme-B sulfoethylthiotransferase activity [GO:0050524] (molecular function) Relationships: is_a alkylthioltransferase activity [GO:0050497] Also known as: coenzyme-B sulphoethylthiotransferase activity, methyl-coenzyme-M reductase activity, 2-(methylthio)ethanesulfonate:N-(7-thioheptanoyl)-3-O-phosphothreonine S-(2-sulfoethyl)thiotransferase activity, methyl coenzyme M reductase activity, methyl-CoM reductase activity Sources: EC:2.8.4.1, RHEA:12532 Definition: Catalysis of the reaction: coenzyme B + methyl-coenzyme M = coenzyme M-coenzyme B heterodisulfide + methane. Methyl-CoM is also known as 2-(methylthio)ethanesulfonate, coenzyme B as N-(7-mercaptoheptanoyl)threonine 3-O-phosphate, and coenzyme M-coenzyme B heterodisulfide as CoM-S-S-CoB.